{
  "gene_name": "Zinc finger protein 107",
  "term_label": "regulation of transcription by RNA polymerase II",
  "term_id": "GO:0006357",
  "gene": "UniProtKB:Q9UII5",
  "gene_symbol": "ZNF107"
}